{
  "term_label": "Unknown biological process",
  "gene_name": "Protein sel-1 homolog 3",
  "gene": "UniProtKB:Q68CR1",
  "term_id": "UNKNOWN:0002",
  "gene_symbol": "SEL1L3"
}